{
  "gene": "UniProtKB:Q9H444",
  "gene_symbol": "CHMP4B",
  "term_id": "GO:0005635",
  "term_label": "nuclear envelope",
  "gene_name": "Charged multivesicular body protein 4b"
}